chromaffin granule amine transport [GO:0015841] (biological process) Definition: The directed movement of amines into, out of or within chromaffin granules. Relationships: is a type of amine transport [GO:0015837] Sources: GOC:mah